{
  "gene_symbol": "GRIK3",
  "term_label": "modulation of chemical synaptic transmission",
  "gene_name": "Glutamate receptor ionotropic, kainate 3",
  "term_id": "GO:0050804",
  "gene": "UniProtKB:Q13003"
}